ventral cord development [GO:0007419] (BP) References: PMID:30826502 Sources: GOC:bf, GOC:go_curators Definition: The process whose specific outcome is the progression of the ventral cord over time, from its formation to the mature structure. The ventral cord is one of the distinguishing traits of the central nervous system of all arthropods (such as insects, crustaceans and arachnids) as well as many other invertebrates, such as the annelid worms. Relationships: is a type of animal organ development [GO:0048513]; is part of central nervous system development [GO:0007417]